{
  "term_label": "nuclear receptor activity",
  "term_id": "GO:0004879",
  "gene_symbol": "HNF4G",
  "gene_name": "Hepatocyte nuclear factor 4-gamma",
  "gene": "UniProtKB:Q14541"
}